{
  "gene_name": "SCO-spondin",
  "gene": "UniProtKB:A2VEC9",
  "term_id": "UNKNOWN:0002",
  "gene_symbol": "SSPOP",
  "term_label": "Unknown biological process"
}